{
  "gene": "UniProtKB:P14543",
  "term_id": "UNKNOWN:0002",
  "term_label": "Unknown biological process",
  "gene_name": "Nidogen-1",
  "gene_symbol": "NID1"
}